polyketide synthase activity [GO:0016218] (molecular function) Definition: Catalysis of a multistep reaction that produce polyketides through decarboxylative condensation of carboxylic acids. The key chain-building reaction, a C-N bond-forming reaction, involves the generation of the characteristic peptide bond by nucleophilic attack of the amino group of an amino-acyl donor unit covalently bound to a downstream peptidyl carrier protein module (amino acyl-S-PCP) on the acyl group of an upstream electrophilic acyl- or peptidyl acyl-S-PCP chain, catalyzed by a condensation (C) domain. Supplementing these core chain-elongation domains are variable numbers of auxiliary domains that are responsible for modification of the growing polypeptide chain by a small set of iterated reactions including epimerization, N-methylation, and heterocyclization. References: PMID:10631508 Relationships: is a type of catalytic activity [GO:0003824]; is part of polyketide biosynthetic process [GO:0030639] Also known as: PKS activity